{
  "gene_name": "Solute carrier family 25 member 33",
  "gene": "UniProtKB:Q9BSK2",
  "gene_symbol": "SLC25A33",
  "term_id": "GO:1990519",
  "term_label": "pyrimidine nucleotide import into mitochondrion"
}